{
  "term_label": "Unknown molecular function",
  "gene_symbol": "EDRF1",
  "gene": "UniProtKB:Q3B7T1",
  "term_id": "UNKNOWN:0001",
  "gene_name": "Erythroid differentiation-related factor 1"
}